positive regulation of glycine secretion, neurotransmission [GO:1904626] (biological process) Definition: Any process that activates or increases the frequency, rate or extent of glycine secretion, neurotransmission. Also known as: up regulation of glycine secretion, neurotransmission, up-regulation of glycine secretion, neurotransmission, upregulation of glycine secretion, neurotransmission, activation of glycine secretion, neurotransmission References: PMID:22988142 Sources: GOC:TermGenie, GO_REF:0000058 Relationships: is a type of positive regulation of neurotransmitter secretion [GO:0001956]; is a type of positive regulation of organic acid transport [GO:0032892]; is a type of positive regulation of amino acid transport [GO:0051957]; is a type of GO:0060094; is a type of regulation of glycine secretion, neurotransmission [GO:1904624]; positively regulates glycine secretion, neurotransmission [GO:0061537]